{
  "term_label": "Unknown biological process",
  "term_id": "UNKNOWN:0002",
  "gene_name": "Putative uncharacterized protein encoded by LINC01554",
  "gene_symbol": "LINC01554",
  "gene": "UniProtKB:Q52M75"
}